{
  "term_id": "GO:0003924",
  "gene_symbol": "RAP2A",
  "gene_name": "Ras-related protein Rap-2a",
  "gene": "UniProtKB:P10114",
  "term_label": "GTPase activity"
}